{
  "term_id": "GO:0000981",
  "term_label": "DNA-binding transcription factor activity, RNA polymerase II-specific",
  "gene": "UniProtKB:Q9Y5J3",
  "gene_symbol": "HEY1",
  "gene_name": "Hairy_enhancer-of-split related with YRPW motif protein 1"
}